carnitine metabolic process [GO:0009437] (biological process) Also known as: carnitine metabolism, vitamin Bt metabolic process, vitamin Bt metabolism Definition: The chemical reactions and pathways involving carnitine (hydroxy-trimethyl aminobutyric acid), a compound that participates in the transfer of acyl groups across the inner mitochondrial membrane. Subtypes: carnitine metabolic process, CoA-linked [GO:0019254], carnitine catabolic process [GO:0042413], carnitine biosynthetic process [GO:0045329] Relationships: is a type of GO:0006577 Sources: GOC:jl, ISBN:0198506732